{
  "gene_name": "Hydroxycarboxylic acid receptor 1",
  "gene": "UniProtKB:Q9BXC0",
  "gene_symbol": "HCAR1",
  "term_label": "plasma membrane",
  "term_id": "GO:0005886"
}